{
  "term_label": "regulation of heart rate by cardiac conduction",
  "gene": "UniProtKB:Q8WWG9",
  "gene_symbol": "KCNE4",
  "term_id": "GO:0086091",
  "gene_name": "Potassium voltage-gated channel subfamily E member 4"
}